{
  "gene": "UniProtKB:Q9Y3Q3",
  "term_id": "GO:0005793",
  "term_label": "endoplasmic reticulum-Golgi intermediate compartment",
  "gene_name": "Transmembrane emp24 domain-containing protein 3",
  "gene_symbol": "TMED3"
}